tryptophan 2-C-methyltransferase activity [GO:0030772] (molecular function) Relationships: is a type of S-adenosylmethionine-dependent methyltransferase activity [GO:0008757] Sources: EC:2.1.1.106, RHEA:17321 Definition: Catalysis of the reaction: S-adenosyl-L-methionine(1+) + L-tryptophan = S-adenosyl-L-homocysteine + L-2-methyltryptophan + H+. Also known as: S-adenosyl-L-methionine:L-tryptophan 2-C-methyltransferase activity, S-adenosylmethionine:tryptophan 2-methyltransferase activity, tryptophan 2-methyltransferase activity